{
  "gene": "UniProtKB:Q99819",
  "gene_name": "Rho GDP-dissociation inhibitor 3",
  "term_id": "GO:0007266",
  "term_label": "Rho protein signal transduction",
  "gene_symbol": "ARHGDIG"
}